{
  "gene": "UniProtKB:P27539",
  "term_id": "GO:0005615",
  "gene_name": "Embryonic growth_differentiation factor 1",
  "gene_symbol": "GDF1",
  "term_label": "extracellular space"
}